maintenance of floral meristem identity [GO:0010076] (biological process) Definition: The process in which an organism retains a population of floral meristem cells, preventing the commitment of all stem cell progeny to a differentiated cell fate. Sources: GOC:dph, GOC:tb Relationships: is a type of maintenance of meristem identity [GO:0010074]